detection of chemical stimulus involved in sensory perception of salty taste [GO:0001583] (biological process) Sources: GOC:go_curators Relationships: is a type of detection of chemical stimulus involved in sensory perception of taste [GO:0050912]; is part of sensory perception of salty taste [GO:0050914] Also known as: perception of salty taste, detection of chemical stimulus, perception of salty taste, sensory transduction of chemical stimulus, salty taste detection, sensory detection of chemical stimulus during perception of salty taste, sensory detection of salty taste, sensory transduction of chemical stimulus during perception of salty taste, sensory transduction of salty taste Definition: The series of events required for a salty taste stimulus to be received and converted to a molecular signal.